transcription initiation at RNA polymerase III promoter [GO:0006384] (BP) Note: Note that promoter clearance is represented as a separate step, not part_of either initiation or elongation. Relationships: is a type of GO:0006352; is part of transcription by RNA polymerase III [GO:0006383] Also known as: transcription initiation from Pol III promoter, transcription initiation from RNA polymerase III promoter, transcription initiation from RNA polymerase III hybrid type promoter, transcription initiation from RNA polymerase III type 1 promoter, transcription initiation from RNA polymerase III type 2 promoter, transcription initiation from RNA polymerase III type 3 promoter Sources: GOC:mah, GOC:txnOH Definition: A transcription initiation process that takes place at a RNA polymerase III gene promoter. Transfer RNAs (tRNA) genes, as well as some other non-coding RNAs, are transcribed by RNA polymerase III.